{
  "gene": "UniProtKB:Q3SY46",
  "term_label": "Unknown cellular component",
  "gene_symbol": "KRTAP13-3",
  "gene_name": "Keratin-associated protein 13-3",
  "term_id": "UNKNOWN:0003"
}